{
  "gene": "UniProtKB:Q15046",
  "gene_name": "Lysine--tRNA ligase",
  "term_label": "ATP:ADP adenylyltransferase activity",
  "term_id": "GO:0003877",
  "gene_symbol": "KARS1"
}